{
  "term_label": "extracellular matrix organization",
  "gene": "UniProtKB:O95980",
  "gene_name": "Reversion-inducing cysteine-rich protein with Kazal motifs",
  "gene_symbol": "RECK",
  "term_id": "GO:0030198"
}